{
  "term_id": "GO:0004888",
  "term_label": "transmembrane signaling receptor activity",
  "gene_symbol": "KIR2DL1",
  "gene_name": "Killer cell immunoglobulin-like receptor 2DL1",
  "gene": "UniProtKB:P43626"
}